propan-2-ol:coenzyme F420 oxidoreductase activity [GO:0052753] (molecular function) References: PMID:15016352, PMID:1879431, PMID:8706724 Sources: GOC:mengo_curators Also known as: F420-dependent secondary alcohol dehydrogenase activity, F420-dependent propan-2-ol dehydrogenase activity, isopropanol:coenzyme F420 oxidoreductase activity Relationships: is a type of oxidoreductase activity, acting on CH-OH group of donors [GO:0016614] Definition: Catalysis of the reaction: propan-2-ol + coenzyme F420 = acetone + reduced coenzyme F420.